modulation of nutrient release by symbiont [GO:0052460] (biological process) Also known as: modulation by host of nutrient release from symbiont Definition: Any process in which an organism modulates the frequency, rate or extent of the release of nutrients from a symbiont organism. The symbiont is defined as the smaller of the organisms involved in a symbiotic interaction. Relationships: is a type of modulation of process of another organism [GO:0035821] Sources: GOC:mtg_pamgo_17jul06 Subtypes: positive regulation of nutrient release by symbiont [GO:0052519]